{
  "gene": "UniProtKB:P09912",
  "term_label": "molecular adaptor activity",
  "term_id": "GO:0060090",
  "gene_symbol": "IFI6",
  "gene_name": "Interferon alpha-inducible protein 6"
}